{
  "term_label": "CCR6 chemokine receptor binding",
  "term_id": "GO:0031731",
  "gene_symbol": "DEFB4B",
  "gene_name": "Defensin beta 4A",
  "gene": "UniProtKB:O15263"
}